{
  "term_label": "MAP kinase kinase kinase activity",
  "gene": "UniProtKB:Q99683",
  "term_id": "GO:0004709",
  "gene_symbol": "MAP3K5",
  "gene_name": "Mitogen-activated protein kinase kinase kinase 5"
}